{
  "term_id": "GO:0005615",
  "gene_name": "Trypsin-2",
  "gene_symbol": "PRSS2",
  "gene": "UniProtKB:P07478",
  "term_label": "extracellular space"
}